hormone binding [GO:0042562] (molecular function) Definition: Binding to an hormone, a naturally occurring substance secreted by specialized cells that affect the metabolism or behavior of cells possessing functional receptors for the hormone. Hormones may be produced by the same, or different, cell as express the receptor. Sources: GOC:jl Relationships: is a type of GO:0005488 Subtypes: androgen binding [GO:0005497], juvenile hormone binding [GO:0005500], auxin binding [GO:0010011], GO:0010331, GO:0010427, peptide hormone binding [GO:0017046], ecdysone binding [GO:0035100], choriogonadotropin hormone binding [GO:0038106], cytokinin binding [GO:0044373], epidermal growth factor binding [GO:0048408], GO:0051379, adiponectin binding [GO:0055100], thyroid hormone binding [GO:0070324], estrogen binding [GO:0099130], GO:1990239